{
  "gene": "UniProtKB:P30532",
  "gene_name": "Neuronal acetylcholine receptor subunit alpha-5",
  "term_label": "synapse",
  "term_id": "GO:0045202",
  "gene_symbol": "CHRNA5"
}